DnaA-oriC complex [GO:1990101] (cellular component) Also known as: DnaA-DNA complex Definition: A protein-DNA complex containing the initiator protein DnaA bound to high-affinity recognition sites in the unique origin of replication, oriC. DnaA-oriC binding is the first step in assembly of a bacterial pre-replicative complex (pre-RC) and is responsible for the timely initiation of replication once per cell cycle. References: PMID:19833870 Sources: GOC:bhm Relationships: is a type of primosome complex [GO:1990077]